{
  "gene_symbol": "ZBTB47",
  "gene_name": "Zinc finger and BTB domain-containing protein 47",
  "term_id": "GO:0000981",
  "term_label": "DNA-binding transcription factor activity, RNA polymerase II-specific",
  "gene": "UniProtKB:Q9UFB7"
}